{
  "gene": "UniProtKB:P62837",
  "term_id": "GO:0005634",
  "gene_name": "Ubiquitin-conjugating enzyme E2 D2",
  "gene_symbol": "UBE2D2",
  "term_label": "nucleus"
}